{
  "gene_symbol": "YAP1",
  "gene_name": "Transcriptional coactivator YAP1",
  "term_id": "GO:0035329",
  "term_label": "hippo signaling",
  "gene": "UniProtKB:P46937"
}